{
  "gene": "UniProtKB:Q9H5V7",
  "gene_symbol": "IKZF5",
  "term_id": "GO:0003700",
  "term_label": "DNA-binding transcription factor activity",
  "gene_name": "Zinc finger protein Pegasus"
}